{
  "term_id": "UNKNOWN:0002",
  "gene_name": "Ras association domain-containing protein 8",
  "gene_symbol": "RASSF8",
  "term_label": "Unknown biological process",
  "gene": "UniProtKB:Q8NHQ8"
}